{
  "gene": "UniProtKB:Q8NCN2",
  "gene_name": "Zinc finger and BTB domain-containing protein 34",
  "term_label": "DNA-binding transcription repressor activity, RNA polymerase II-specific",
  "term_id": "GO:0001227",
  "gene_symbol": "ZBTB34"
}